{
  "gene_name": "GRB2-associated-binding protein 2",
  "term_id": "GO:0005068",
  "gene": "UniProtKB:Q9UQC2",
  "term_label": "transmembrane receptor protein tyrosine kinase adaptor activity",
  "gene_symbol": "GAB2"
}